vitamin E binding [GO:0008431] (molecular function) Definition: Binding to a vitamin E, tocopherol, which includes a series of eight structurally similar compounds. Alpha-tocopherol is the most active form in humans and is a powerful biological antioxidant. Sources: ISBN:0721662544 Also known as: tocopherol binding, alpha-tocopherol binding Relationships: is a type of vitamin binding [GO:0019842]; is a type of GO:1901363